{
  "gene": "UniProtKB:Q9NSK7",
  "term_label": "Unknown cellular component",
  "gene_symbol": "C19orf12",
  "term_id": "UNKNOWN:0003",
  "gene_name": "Protein C19orf12"
}